thymine dehydrogenase activity [GO:0052620] (molecular function) Relationships: is a type of oxidoreductase activity, acting on CH or CH2 groups [GO:0016725] Definition: Catalysis of the reaction: H2O + thymine + acceptor = 5-methyl-barbiturate + donor-H2. Sources: RHEA:13469